{
  "gene_symbol": "RNF40",
  "term_id": "UNKNOWN:0002",
  "gene_name": "E3 ubiquitin-protein ligase BRE1B",
  "gene": "UniProtKB:O75150",
  "term_label": "Unknown biological process"
}